blood vessel endothelial cell migration [GO:0043534] (biological process) References: PMID:11166264 Relationships: is a type of GO:0043542 Subtypes: cell migration involved in sprouting angiogenesis [GO:0002042], GO:0002044, venous endothelial cell migration involved in lymph vessel development [GO:0060855] Definition: The orderly movement of an endothelial cell into the extracellular matrix in order to form new blood vessels during angiogenesis. Regulation: regulated by regulation of blood vessel endothelial cell migration [GO:0043535]; positively regulated by positive regulation of blood vessel endothelial cell migration [GO:0043536]; negatively regulated by negative regulation of blood vessel endothelial cell migration [GO:0043537]